{
  "gene": "UniProtKB:Q96S66",
  "term_id": "UNKNOWN:0002",
  "gene_name": "Chloride channel CLIC-like protein 1",
  "term_label": "Unknown biological process",
  "gene_symbol": "CLCC1"
}